{
  "term_id": "GO:0043161",
  "gene_name": "Ataxin-3",
  "gene_symbol": "ATXN3",
  "term_label": "proteasome-mediated ubiquitin-dependent protein catabolic process",
  "gene": "UniProtKB:P54252"
}